leukocyte cell-cell adhesion [GO:0007159] (biological process) Definition: The attachment of a leukocyte to another cell via adhesion molecules. Sources: GOC:go_curators Also known as: leukocyte adhesion, leukocyte cell adhesion Relationships: is a type of cell-cell adhesion [GO:0098609] Subtypes: leukocyte adhesion to vascular endothelial cell [GO:0061756], leukocyte aggregation [GO:0070486], B cell adhesion [GO:0097323] Regulation: regulated by regulation of leukocyte cell-cell adhesion [GO:1903037]; negatively regulated by negative regulation of leukocyte cell-cell adhesion [GO:1903038]; positively regulated by positive regulation of leukocyte cell-cell adhesion [GO:1903039]